(+)-menthofuran synthase activity [GO:0052582] (MF) Also known as: (+)-MFS activity, (+)-pulegone 9-hydroxylase activity, (+)-pulegone,NADPH:oxygen oxidoreductase (9-hydroxylating) activity, cytochrome P450 menthofuran synthase activity, menthofuran synthase activity Definition: Catalysis of the reaction: (R)-pulegone + reduced [NADPH--hemoprotein reductase] + O2 = (R)-menthofuran + 2 H2O + +H+ + oxidized [NADPH--hemoprotein reductase]. Relationships: is a type of oxidoreductase activity, acting on paired donors, with incorporation or reduction of molecular oxygen, reduced flavin or flavoprotein as one donor, and incorporation of one atom of oxygen [GO:0016712] Sources: RHEA:25658